{
  "gene": "UniProtKB:Q6SA08",
  "term_label": "Unknown biological process",
  "gene_name": "Testis-specific serine_threonine-protein kinase 4",
  "term_id": "UNKNOWN:0002",
  "gene_symbol": "TSSK4"
}